cell-cell signaling [GO:0007267] (biological process) Also known as: cell-cell signalling Subtypes: mesodermal-endodermal cell signaling [GO:0003131], endodermal-mesodermal cell signaling [GO:0003133], gamma-aminobutyric acid signaling pathway [GO:0007214], visceral mesoderm-endoderm interaction involved in midgut development [GO:0007495], ectoderm and mesoderm interaction [GO:0007499], quorum sensing [GO:0009372], determination of muscle attachment site [GO:0016204], cerebellar Purkinje cell-granule cell precursor cell signaling [GO:0021937], autocrine signaling [GO:0035425], paracrine signaling [GO:0038001], endocrine signaling [GO:0038002], GO:0044345, cell-cell signaling involved in cell fate commitment [GO:0045168], cell-cell signaling involved in lung development [GO:0060495], mesenchymal-endodermal cell signaling [GO:0060497], mesenchymal-epithelial cell signaling [GO:0060638], regulation of branching involved in mammary cord morphogenesis by fat precursor cell-epithelial cell signaling [GO:0060656], regulation of mammary gland cord elongation by mammary fat precursor cell-epithelial cell signaling [GO:0060657], cell-cell signaling involved in placenta development [GO:0060673], epithelial-mesenchymal cell signaling [GO:0060684], cell-cell signaling involved in mammary gland development [GO:0060764], epiblast cell-extraembryonic ectoderm cell signaling [GO:0060802], cell-cell signaling involved in kidney development [GO:0060995], c-di-GMP signaling [GO:0061939], GO:0072043, cell-cell signaling involved in cardiac conduction [GO:0086019], GO:0099156, GO:0099536, polyphosphate-mediated signaling [GO:0110094], oscillatory cAMP signaling [GO:0140676], glial cell-neuron signaling [GO:0150098], GO:0150099 Definition: Any process that mediates the transfer of information from one cell to another. This process includes signal transduction in the receiving cell and, where applicable, release of a ligand and any processes that actively facilitate its transport and presentation to the receiving cell. Examples include signaling via soluble ligands, via cell adhesion molecules and via gap junctions. Relationships: is a type of GO:0007154; is_a signaling [GO:0023052] Sources: GOC:dos, GOC:mah